{
  "term_id": "UNKNOWN:0002",
  "gene_symbol": "ZNF45",
  "term_label": "Unknown biological process",
  "gene": "UniProtKB:Q02386",
  "gene_name": "Zinc finger protein 45"
}